{
  "gene_name": "Glycerophosphocholine phosphodiesterase GPCPD1",
  "term_id": "GO:0047389",
  "gene_symbol": "GPCPD1",
  "gene": "UniProtKB:Q9NPB8",
  "term_label": "glycerophosphocholine phosphodiesterase activity"
}